{
  "term_label": "ubiquitin protein ligase activity",
  "gene_name": "E3 ubiquitin-protein ligase synoviolin",
  "gene": "UniProtKB:Q86TM6",
  "gene_symbol": "SYVN1",
  "term_id": "GO:0061630"
}